{
  "gene": "UniProtKB:P38405",
  "term_label": "adenylate cyclase-activating dopamine receptor signaling pathway",
  "term_id": "GO:0007191",
  "gene_name": "Guanine nucleotide-binding protein G(olf) subunit alpha",
  "gene_symbol": "GNAL"
}